{
  "gene_name": "Abasic site processing protein HMCES",
  "gene_symbol": "HMCES",
  "term_label": "protein-DNA covalent cross-linking activity",
  "gene": "UniProtKB:Q96FZ2",
  "term_id": "GO:0160129"
}